{
  "gene_name": "(Lyso)-N-acylphosphatidylethanolamine lipase",
  "gene": "UniProtKB:Q8TB40",
  "term_id": "GO:0006654",
  "gene_symbol": "ABHD4",
  "term_label": "phosphatidic acid biosynthetic process"
}